lamellipodium assembly involved in ameboidal cell migration [GO:0003363] (biological process) Subtypes: lamellipodium assembly involved in mesendodermal cell migration [GO:0003364] Sources: GOC:ascb_2009, GOC:dph, GOC:tb Relationships: is a type of GO:0030032; is part of GO:0001667 Definition: Formation of a lamellipodium, a thin sheetlike extension of the surface of a migrating cell that contributes to the directed self propelled movement of a cell.